Golgi distribution to daughter cells [GO:0090167] (biological process) Sources: GOC:ascb_2009, GOC:dph, GOC:tb Also known as: Golgi apparatus distribution to daughter cells Relationships: is a type of GO:0007030; is a type of Golgi localization [GO:0051645]; is part of Golgi inheritance [GO:0048313] Definition: Any process in which disassembled Golgi vesicles are localized into daughter cells upon cell division.